{
  "gene": "UniProtKB:Q15973",
  "term_id": "GO:0000981",
  "gene_symbol": "ZNF124",
  "term_label": "DNA-binding transcription factor activity, RNA polymerase II-specific",
  "gene_name": "Zinc finger protein 124"
}